diaminopimelate epimerase activity [GO:0008837] (MF) Definition: Catalysis of the reaction: LL-2,6-diaminopimelate = meso-2,6-diaminopimelate. Also known as: LL-2,6-diaminoheptanedioate 2-epimerase activity Sources: EC:5.1.1.7, RHEA:15393 Relationships: is a type of amino-acid racemase activity [GO:0047661]